{
  "term_label": "Unknown biological process",
  "gene": "UniProtKB:Q8NGL6",
  "gene_name": "Olfactory receptor 4A15",
  "term_id": "UNKNOWN:0002",
  "gene_symbol": "OR4A15"
}